glucose-6-phosphate transmembrane transporter activity [GO:0015152] (molecular function) Subtypes: glucose 6-phosphate:phosphate antiporter activity [GO:0061513] Sources: GOC:ai, GOC:mtg_transport, ISBN:0815340729 Relationships: is a type of hexose phosphate transmembrane transporter activity [GO:0015119]; is part of glucose-6-phosphate transport [GO:0015760] Definition: Enables the transfer of glucose-6-phosphate from one side of a membrane to the other. Glucose-6-phosphate is a monophosphorylated derivative of glucose with the phosphate group attached to C-6.